cytoplasmic microtubule organization [GO:0031122] (biological process) Definition: A process that is carried out at the cellular level which results in the assembly, arrangement of constituent parts, or disassembly of structures formed of microtubules and associated proteins in the cytoplasm of a cell. Subtypes: GO:0010938, astral microtubule organization [GO:0030953], cortical microtubule organization [GO:0043622] Sources: GOC:mah Also known as: cytoplasmic microtubule organisation, cytoplasmic microtubule organization and biogenesis Relationships: is a type of GO:0000226; is a type of supramolecular fiber organization [GO:0097435]